{
  "term_id": "UNKNOWN:0003",
  "gene_name": "2-(3-amino-3-carboxypropyl)histidine synthase subunit 1",
  "term_label": "Unknown cellular component",
  "gene": "UniProtKB:Q9BZG8",
  "gene_symbol": "DPH1"
}